{
  "gene": "UniProtKB:Q9Y651",
  "gene_symbol": "SOX21",
  "term_id": "GO:0000122",
  "gene_name": "Transcription factor SOX-21",
  "term_label": "negative regulation of transcription by RNA polymerase II"
}